regulation of alpha-beta T cell proliferation [GO:0046640] (biological process) Subtypes: GO:0046641, negative regulation of alpha-beta T cell proliferation [GO:0046642], GO:0051140, regulation of CD4-positive, alpha-beta T cell proliferation [GO:2000561], regulation of CD8-positive, alpha-beta T cell proliferation [GO:2000564] Relationships: is a type of regulation of T cell proliferation [GO:0042129]; is a type of regulation of alpha-beta T cell activation [GO:0046634]; regulates alpha-beta T cell proliferation [GO:0046633] Definition: Any process that modulates the frequency, rate or extent of alpha-beta T cell proliferation. Also known as: regulation of alpha-beta T lymphocyte proliferation, regulation of alpha-beta T-cell proliferation, regulation of alpha-beta T-lymphocyte proliferation Sources: GOC:ai